{
  "term_label": "Unknown molecular function",
  "gene_name": "Retroviral-like aspartic protease 1",
  "term_id": "UNKNOWN:0001",
  "gene": "UniProtKB:Q53RT3",
  "gene_symbol": "ASPRV1"
}